{
  "gene_symbol": "RERGL",
  "term_id": "UNKNOWN:0002",
  "term_label": "Unknown biological process",
  "gene_name": "Ras-related and estrogen-regulated growth inhibitor-like protein",
  "gene": "UniProtKB:Q9H628"
}